{
  "gene": "UniProtKB:P43356",
  "term_label": "negative regulation of transcription by RNA polymerase II",
  "gene_name": "Melanoma-associated antigen 2",
  "gene_symbol": "MAGEA2B",
  "term_id": "GO:0000122"
}